antennal morphogenesis [GO:0048800] (biological process) Sources: GOC:jid Definition: The process in which the anatomical structures of the antenna are generated and organized. Relationships: is a type of post-embryonic animal morphogenesis [GO:0009886]; is a type of GO:0035107; is part of eye-antennal disc morphogenesis [GO:0007455]; is part of GO:0007469